{
  "gene_symbol": "NODAL",
  "term_id": "GO:0005125",
  "gene_name": "Nodal homolog",
  "term_label": "cytokine activity",
  "gene": "UniProtKB:Q96S42"
}